{
  "gene_name": "Uncharacterized protein C9orf43",
  "gene": "UniProtKB:Q8TAL5",
  "term_label": "Unknown cellular component",
  "gene_symbol": "C9orf43",
  "term_id": "UNKNOWN:0003"
}